4-amino-5-hydroxymethyl-2-methylpyrimidine diphosphatase activity [GO:0002145] (molecular function) Definition: Catalysis of the reaction: 4-amino-5-hydroxymethyl-2-methylpyrimidine pyrophosphate + H2O = hydroxymethylpyrimidine phosphate + phosphate + H+. Relationships: is a type of pyrophosphatase activity [GO:0016462] Also known as: HMP-PP diphosphatase, HMP-PP pyrophosphatase Sources: MetaCyc:RXN0-3543